histamine secretion by mast cell [GO:0002553] (biological process) Definition: The regulated release of histamine by a mast cell or group of mast cells. Sources: GOC:add, ISBN:0781735149 Relationships: is a type of histamine secretion involved in inflammatory response [GO:0002441]; is a type of establishment of localization in cell [GO:0051649]; is a type of exocytic process [GO:0140029]; is part of mast cell degranulation [GO:0043303] Regulation: regulated by regulation of histamine secretion by mast cell [GO:1903593]; negatively regulated by negative regulation of histamine secretion by mast cell [GO:1903594]; positively regulated by positive regulation of histamine secretion by mast cell [GO:1903595]